habituation [GO:0046959] (biological process) Definition: A decrease in a behavioral response to a repeated stimulus. This is exemplified by the failure of a person to show a startle response to a loud noise that has been repeatedly presented. Sources: ISBN:0582227089 Relationships: is a type of GO:0046958